{
  "term_id": "GO:0061617",
  "gene_symbol": "CHCHD3",
  "term_label": "MICOS complex",
  "gene": "UniProtKB:Q9NX63",
  "gene_name": "MICOS complex subunit MIC19"
}